{
  "gene_name": "Mitogen-activated protein kinase 14",
  "gene_symbol": "MAPK14",
  "gene": "UniProtKB:Q16539",
  "term_label": "nucleus",
  "term_id": "GO:0005634"
}